cyclooxygenase pathway [GO:0019371] (biological process) Definition: The chemical reactions and pathways by which prostaglandins are formed from arachidonic acid, and in which prostaglandin-endoperoxide synthase (cyclooxygenase) catalyzes the committed step in the conversion of arachidonic acid to the prostaglandin-endoperoxides PGG2 and PGH2. References: PMID:19854273 Relationships: is a type of GO:0019369; BFO_0000050 GO:0001516